spindle assembly checkpoint signaling [GO:0071173] (biological process) Also known as: SAC, signal transduction involved in spindle assembly checkpoint, spindle assembly checkpoint Note: Note that this term should not be used for direct manual annotation as it should always be possible to specify the type of spindle assembly checkpoint (mitotic or meiotic). Definition: A signaling process that delays the metaphase/anaphase transition until the spindle is correctly assembled and chromosomes are attached to the spindle. Relationships: is a type of GO:0031577 Subtypes: GO:0007094, meiotic spindle assembly checkpoint signaling [GO:0033316] Sources: GOC:mah